{
  "term_id": "GO:0061630",
  "gene": "UniProtKB:Q496Y0",
  "term_label": "ubiquitin protein ligase activity",
  "gene_name": "LON peptidase N-terminal domain and RING finger protein 3",
  "gene_symbol": "LONRF3"
}